MH1 domain binding [GO:0035501] (molecular function) Relationships: is a type of GO:0019904 Also known as: MAD homology 1 domain binding Definition: Binding to a MH1 (MAD homology 1) protein domain. The MH1 domain is found at the amino terminus of MAD related proteins such as Smads and can mediate DNA binding in some proteins. Smads also use the MH1 domain to interact with some transcription factors. Sources: Pfam:PF03165